{
  "gene_name": "H(+)_Cl(-) exchange transporter 4",
  "gene_symbol": "CLCN4",
  "term_label": "synaptic vesicle",
  "gene": "UniProtKB:P51793",
  "term_id": "GO:0008021"
}